{
  "gene_name": "Small integral membrane protein 23",
  "term_label": "Unknown biological process",
  "term_id": "UNKNOWN:0002",
  "gene": "UniProtKB:A6NLE4",
  "gene_symbol": "SMIM23"
}